{
  "term_label": "Unknown cellular component",
  "gene_symbol": "TTTY13",
  "gene": "UniProtKB:Q9BZ97",
  "term_id": "UNKNOWN:0003",
  "gene_name": "Putative transcript Y 13 protein"
}